{
  "gene_symbol": "FCSK",
  "gene": "UniProtKB:Q8N0W3",
  "gene_name": "L-fucose kinase",
  "term_label": "fucokinase activity",
  "term_id": "GO:0050201"
}